negative regulation of filamentous growth of a population of unicellular organisms in response to pH [GO:1900742] (biological process) Also known as: down regulation of filamentous growth of a population of unicellular organisms in response to pH, down-regulation of filamentous growth of a population of unicellular organisms in response to pH, downregulation of filamentous growth of a population of unicellular organisms in response to pH, inhibition of filamentous growth of a population of unicellular organisms in response to pH Subtypes: negative regulation of filamentous growth of a population of unicellular organisms in response to neutral pH [GO:1900441] Sources: GOC:TermGenie, GOC:di Definition: Any process that stops, prevents or reduces the frequency, rate or extent of filamentous growth of a population of unicellular organisms in response to pH. Relationships: is a type of negative regulation of response to stimulus [GO:0048585]; is a type of negative regulation of filamentous growth of a population of unicellular organisms [GO:1900429]; is a type of GO:1900741; negatively regulates filamentous growth of a population of unicellular organisms in response to pH [GO:0036177]